{
  "gene_name": "Intraflagellar transport protein 20 homolog",
  "term_label": "intraciliary transport particle",
  "gene_symbol": "IFT20",
  "gene": "UniProtKB:Q8IY31",
  "term_id": "GO:0030990"
}